{
  "term_label": "cytoplasm",
  "gene_name": "Adenylate kinase 7",
  "gene_symbol": "AK7",
  "term_id": "GO:0005737",
  "gene": "UniProtKB:Q96M32"
}